{
  "gene_symbol": "SAP30L",
  "term_label": "regulation of DNA-templated transcription",
  "term_id": "GO:0006355",
  "gene_name": "Histone deacetylase complex subunit SAP30L",
  "gene": "UniProtKB:Q9HAJ7"
}